Ost-alpha/Ost-beta complex [GO:0044731] (cellular component) Relationships: is_a plasma membrane protein complex [GO:0098797] Also known as: Ost alpha-Ost beta complex, SLC51 complex, (Ost)2 complex References: PMID:17650074, PMID:22535958 Definition: A heterodimeric protein complex composed of Ost-alpha/SLC51A and Ost-beta/SLC51B subunits and involved in bile acid transport activity.